{
  "gene_symbol": "BTBD10",
  "gene": "UniProtKB:Q9BSF8",
  "gene_name": "BTB_POZ domain-containing protein 10",
  "term_label": "cytoplasm",
  "term_id": "GO:0005737"
}